{
  "term_label": "nucleus",
  "gene_name": "DNA repair and recombination protein RAD54-like",
  "term_id": "GO:0005634",
  "gene_symbol": "RAD54L",
  "gene": "UniProtKB:Q92698"
}